{
  "gene_symbol": "POU3F1",
  "term_id": "GO:0000978",
  "term_label": "RNA polymerase II cis-regulatory region sequence-specific DNA binding",
  "gene_name": "POU domain, class 3, transcription factor 1",
  "gene": "UniProtKB:Q03052"
}